catecholamine metabolic process [GO:0006584] (biological process) Also known as: catecholamine metabolism Regulation: regulated by GO:0042069 Relationships: is a type of biogenic amine metabolic process [GO:0006576]; is a type of catechol-containing compound metabolic process [GO:0009712] Subtypes: epinephrine metabolic process [GO:0042414], norepinephrine metabolic process [GO:0042415], dopamine metabolic process [GO:0042417], catecholamine biosynthetic process [GO:0042423], catecholamine catabolic process [GO:0042424] Sources: GOC:jl, ISBN:0198506732 Definition: The chemical reactions and pathways involving any of a group of physiologically important biogenic amines that possess a catechol (3,4-dihydroxyphenyl) nucleus and are derivatives of 3,4-dihydroxyphenylethylamine.